{
  "gene": "UniProtKB:Q8N3U4",
  "gene_symbol": "STAG2",
  "gene_name": "Cohesin subunit SA-2",
  "term_label": "cohesin complex",
  "term_id": "GO:0008278"
}